histone deacetylase activity, NAD-dependent [GO:0017136] (molecular function) Definition: Catalysis of the reaction: N(6)-acetyl-L-lysyl-[histone] + NAD+ + H2O = L-lysyl-[protein] + 2''-O-acetyl-ADP-D-ribose + nicotinamide. This reaction transfers an acetyl group from a histone to NAD, producing nicotinamide. Also known as: histone deacetylase activity, NAD-dependent histone deacetylase activity, NAD-dependent histone lysine deacetylase activity, sirtuin, SIR2 Subtypes: histone H3K14 deacetylase activity, NAD-dependent [GO:0032041], histone H3K9 deacetylase activity, NAD-dependent [GO:0046969], GO:0046970, histone H3K18 deacetylase activity, NAD-dependent [GO:0097372], GO:0140765, GO:0141222 Note: Histone deacytylase (HDAC) enzymes are divided into four classes: the Class I Rpd3-like proteins (in human: HDAC1, HDAC2, HDAC3, and HDAC8); the Class II Hda1-like proteins (in human: HDAC4, HDAC5, HDAC6, HDAC7, HDAC9, and HDAC10); the Class III Sir2-like proteins (in human: SIRT1, SIRT2, SIRT3, SIRT4, SIRT5, SIRT6, and SIRT7); and the Class IV protein (HDAC11 in human). Except for Class III enzymes, the mechanism is a metal-dependent hydrolysis of the acetylated substrate. The Class III HDACs use NAD+ as a reactant to deacetylate acetyl lysine residues of protein substrates forming nicotinamide, the deacetylated product, and the metabolite 2'-O-acetyl-ADP-ribose. Therefore, Class III are classified as transferases (EC:2) and others are hydrolases (EC:3). References: PMID:24691964, PMID:28450737 Relationships: is_a histone deacetylase activity [GO:0004407]; is a type of NAD-dependent protein lysine deacetylase activity [GO:0034979]